{
  "gene_name": "Astrotactin-1",
  "gene_symbol": "ASTN1",
  "gene": "UniProtKB:O14525",
  "term_label": "neuron cell-cell adhesion",
  "term_id": "GO:0007158"
}